host cell membrane [GO:0033644] (cellular component) Subtypes: host cell plasma membrane [GO:0020002], host cell endomembrane system [GO:0033645], host thylakoid membrane [GO:0044160], GO:0044162, GO:0044167, host cell endoplasmic reticulum-Golgi intermediate compartment membrane [GO:0044173], GO:0044175, host cell Golgi membrane [GO:0044178], GO:0044188, GO:0044191, host cell nuclear membrane [GO:0044200], host outer membrane [GO:0044384], extrahaustorial membrane [GO:0085037], hyphal membrane [GO:0085039], GO:0085042 Relationships: is a type of host cell part [GO:0033643] Definition: Double layer of lipid molecules as it encloses host cells, and, in eukaryotes, many organelles; may be a single or double lipid bilayer; also includes associated proteins. The host is defined as the larger of the organisms involved in a symbiotic interaction. Sources: GOC:pamgo_curators